{
  "term_id": "GO:0050911",
  "gene_symbol": "OR10K1",
  "gene_name": "Olfactory receptor 10K1",
  "gene": "UniProtKB:Q8NGX5",
  "term_label": "detection of chemical stimulus involved in sensory perception of smell"
}